{
  "gene_name": "Protein shisa-6",
  "term_label": "postsynaptic membrane",
  "gene_symbol": "SHISA6",
  "term_id": "GO:0045211",
  "gene": "UniProtKB:Q6ZSJ9"
}